mandelamide amidase activity [GO:0050537] (molecular function) Sources: EC:3.5.1.86, RHEA:22876 Definition: Catalysis of the reaction: (R)-mandelamide + H2O = (R)-mandelate + NH4. Relationships: is a type of hydrolase activity, acting on carbon-nitrogen (but not peptide) bonds, in linear amides [GO:0016811] Also known as: Pseudomonas mandelamide hydrolase activity, mandelamide hydrolase activity